{
  "term_label": "plasma membrane",
  "gene_name": "Sprouty-related, EVH1 domain-containing protein 3",
  "gene_symbol": "SPRED3",
  "gene": "UniProtKB:Q2MJR0",
  "term_id": "GO:0005886"
}